{
  "term_id": "UNKNOWN:0001",
  "gene_symbol": "PRR15",
  "gene": "UniProtKB:Q8IV56",
  "term_label": "Unknown molecular function",
  "gene_name": "Proline-rich protein 15"
}